{
  "gene_symbol": "GYPC",
  "gene": "UniProtKB:P04921",
  "term_label": "Unknown biological process",
  "gene_name": "Glycophorin-C",
  "term_id": "UNKNOWN:0002"
}